{
  "gene": "UniProtKB:Q99417",
  "term_id": "GO:0003713",
  "gene_name": "c-Myc-binding protein",
  "term_label": "transcription coactivator activity",
  "gene_symbol": "MYCBP"
}